embryonic forelimb morphogenesis [GO:0035115] (biological process) Definition: The process, occurring in the embryo, by which the anatomical structures of the forelimb are generated and organized. The forelimbs are the front limbs of an animal, e.g. the arms of a human. Sources: ISBN:0198612001 Also known as: embryonic arm morphogenesis Relationships: is a type of GO:0030326; is a type of forelimb morphogenesis [GO:0035136]